{
  "gene": "UniProtKB:Q8TAX0",
  "term_id": "GO:0007389",
  "gene_symbol": "OSR1",
  "term_label": "pattern specification process",
  "gene_name": "Protein odd-skipped-related 1"
}